{
  "gene_name": "Aldo-keto reductase family 1 member D1",
  "term_label": "cytosol",
  "term_id": "GO:0005829",
  "gene": "UniProtKB:P51857",
  "gene_symbol": "AKR1D1"
}